negative regulation of neuromuscular synaptic transmission [GO:1900074] (biological process) Relationships: is a type of GO:0050805; is a type of GO:1900073; negatively regulates GO:0007274 Sources: GOC:TermGenie, GOC:kmv Definition: Any process that stops, prevents or reduces the frequency, rate or extent of neuromuscular synaptic transmission. Also known as: down regulation of neuromuscular synaptic transmission, down-regulation of neuromuscular synaptic transmission, downregulation of neuromuscular synaptic transmission, inhibition of neuromuscular synaptic transmission